{
  "term_id": "GO:0007179",
  "gene": "UniProtKB:P10600",
  "gene_symbol": "TGFB3",
  "term_label": "transforming growth factor beta receptor signaling pathway",
  "gene_name": "Transforming growth factor beta-3 proprotein"
}